{
  "gene_name": "Fanconi anemia group D2 protein",
  "term_label": "double-strand break repair involved in meiotic recombination",
  "term_id": "GO:1990918",
  "gene_symbol": "FANCD2",
  "gene": "UniProtKB:Q9BXW9"
}